response to differentiation-inducing factor 1 [GO:1903013] (BP) Definition: Any process that results in a change in state or activity of a cell or an organism (in terms of movement, secretion, enzyme production, gene expression, etc.) as a result of a 1-(3,5-dichloro-2,6-dihydroxy-4-methoxyphenyl)hexan-1-one stimulus. References: PMID:22365144 Sources: GOC:TermGenie, GO_REF:0000071 Also known as: response to 1-(3,5-dichloro-2,6-dihydroxy-4-methoxyphenyl)hexan-1-one, DIF-1, response to DIF-1, response to DIF1 Relationships: is a type of GO:0045472; is_a response to ketone [GO:1901654] Subtypes: cellular response to differentiation-inducing factor 1 [GO:1903014]